{
  "term_id": "GO:1902358",
  "gene": "UniProtKB:P58743",
  "gene_name": "Prestin",
  "term_label": "sulfate transmembrane transport",
  "gene_symbol": "SLC26A5"
}